aminoglycoside 2'-N-acetyltransferase activity [GO:0047921] (molecular function) Also known as: acetyl-CoA:gentamicin-C1a N2'-acetyltransferase activity, acetyl-CoA:gentamycin-C1a N2'-acetyltransferase activity, gentamicin 2'-N-acetyltransferase activity, gentamicin acetyltransferase II activity, gentamycin 2'-N-acetyltransferase activity, gentamycin acetyltransferase II Sources: EC:2.3.1.59, RHEA:24516 Definition: Catalysis of the reaction: acetyl-CoA + gentamicin C(1a) = N(2')-acetylgentamicin C(1a) + CoA + H+. This is acetylation of the 2'-amino group of the 6-deoxy-6-aminoglucose ring. Relationships: is a type of GO:0034069